{
  "gene_symbol": "NUP155",
  "term_label": "nuclear pore inner ring",
  "term_id": "GO:0044611",
  "gene": "UniProtKB:O75694",
  "gene_name": "Nuclear pore complex protein Nup155"
}